lateral ganglionic eminence cell proliferation [GO:0022018] (biological process) Definition: The multiplication or reproduction of lateral ganglionic eminence cells, resulting in the expansion of the cell population. Sources: GOC:cls, GOC:dgh, GOC:dph, GOC:jid, GO_REF:0000021 Relationships: is a type of subpallium cell proliferation in forebrain [GO:0022012]